{
  "gene_symbol": "SLC4A5",
  "term_label": "plasma membrane",
  "term_id": "GO:0005886",
  "gene": "UniProtKB:Q9BY07",
  "gene_name": "Electrogenic sodium bicarbonate cotransporter 4"
}